vacuolar localization [GO:1990849] (biological process) Also known as: maintenance of vacuolar localization, maintenance of vacuole localization, maintenance of vacuole location, maintenance of vacuolar location Relationships: is_a organelle localization [GO:0051640] References: PMID:26283797 Subtypes: lysosome localization [GO:0032418], GO:0061906, GO:0140027, vacuole-ER tethering [GO:1990854] Definition: Any process in which the vacuole is transported to, and/or maintained in, a specific location within the cell.